L-arabinonolactonase activity [GO:0050021] (MF) Definition: Catalysis of the reaction: L-arabinono-1,4-lactone + H2O = L-arabinonate + H+. Also known as: L-arabinono-1,4-lactone lactonohydrolase activity Relationships: is a type of carboxylic ester hydrolase activity [GO:0052689] Sources: EC:3.1.1.15, RHEA:16217